{
  "term_id": "GO:0030036",
  "gene": "UniProtKB:Q9Y6W5",
  "gene_name": "Actin-binding protein WASF2",
  "gene_symbol": "WASF2",
  "term_label": "actin cytoskeleton organization"
}